{
  "gene": "UniProtKB:Q49A92",
  "gene_name": "Uncharacterized protein C8orf34",
  "term_id": "UNKNOWN:0002",
  "term_label": "Unknown biological process",
  "gene_symbol": "C8orf34"
}